{
  "gene_symbol": "RND1",
  "gene": "UniProtKB:Q92730",
  "term_id": "GO:0007165",
  "gene_name": "Rho-related GTP-binding protein Rho6",
  "term_label": "signal transduction"
}